{
  "gene": "UniProtKB:O75394",
  "gene_symbol": "MRPL33",
  "term_label": "Unknown biological process",
  "term_id": "UNKNOWN:0002",
  "gene_name": "Large ribosomal subunit protein bL33m"
}